{
  "gene": "UniProtKB:Q9Y5B0",
  "term_id": "UNKNOWN:0003",
  "gene_symbol": "CTDP1",
  "term_label": "Unknown cellular component",
  "gene_name": "RNA polymerase II subunit A C-terminal domain phosphatase"
}